{
  "gene": "UniProtKB:O75674",
  "term_id": "GO:0005768",
  "gene_symbol": "TOM1L1",
  "gene_name": "TOM1-like protein 1",
  "term_label": "endosome"
}